interferon-omega production [GO:0072653] (BP) Relationships: is a type of GO:0032606 Note: Note that this term is in the subset of terms that should not be used for direct gene product annotation. Instead, select one of the 'regulation' children terms. References: PMID:15546383 Sources: GOC:BHF, GOC:mah Definition: The appearance of interferon-omega due to biosynthesis or secretion following a cellular stimulus, resulting in an increase in its intracellular or extracellular levels. Also known as: IFN-omega production, IFNW production, interferon-omega secretion